microneme membrane [GO:0033163] (cellular component) Definition: The lipid bilayer surrounding a microneme. Sources: GOC:mah Relationships: is a type of bounding membrane of organelle [GO:0098588]; is part of GO:0020009